regulation of modification of synaptic structure [GO:1905244] (BP) Definition: Any process that modulates the frequency, rate or extent of modification of synaptic structure. Relationships: is a type of regulation of synapse organization [GO:0050807]; regulates modification of synaptic structure [GO:0099563] Subtypes: regulation of modification of synapse structure, modulating synaptic transmission [GO:0098987], regulation of modification of postsynaptic structure [GO:0099159] References: PMID:25164660 Sources: GOC:TermGenie, GO_REF:0000058 Also known as: regulation of synapse remodelling